{
  "gene": "UniProtKB:A6NGB9",
  "gene_name": "WAS_WASL-interacting protein family member 3",
  "gene_symbol": "WIPF3",
  "term_label": "retrograde transport, endosome to Golgi",
  "term_id": "GO:0042147"
}